{
  "term_id": "GO:0000164",
  "term_label": "protein phosphatase type 1 complex",
  "gene_symbol": "PPP1R3G",
  "gene": "UniProtKB:B7ZBB8",
  "gene_name": "Protein phosphatase 1 regulatory subunit 3G"
}